{
  "gene_symbol": "ALDH3A2",
  "gene": "UniProtKB:P51648",
  "term_label": "aldehyde metabolic process",
  "term_id": "GO:0006081",
  "gene_name": "Aldehyde dehydrogenase family 3 member A2"
}